{
  "gene_name": "BEN domain-containing protein 4",
  "gene_symbol": "BEND4",
  "term_id": "UNKNOWN:0003",
  "gene": "UniProtKB:Q6ZU67",
  "term_label": "Unknown cellular component"
}